{
  "term_id": "GO:0006364",
  "term_label": "rRNA processing",
  "gene_symbol": "UTP15",
  "gene_name": "U3 small nucleolar RNA-associated protein 15 homolog",
  "gene": "UniProtKB:Q8TED0"
}